{
  "gene_name": "Protein-cysteine N-palmitoyltransferase HHAT",
  "term_label": "endoplasmic reticulum",
  "gene": "UniProtKB:Q5VTY9",
  "term_id": "GO:0005783",
  "gene_symbol": "HHAT"
}